{
  "gene_symbol": "ATXN2",
  "term_label": "mRNA binding",
  "gene": "UniProtKB:Q99700",
  "gene_name": "Ataxin-2",
  "term_id": "GO:0003729"
}